ribosome-associated ubiquitin-dependent protein catabolic process [GO:1990116] (biological process) Also known as: RAD, ribosome-associated degradation, ribosome-associated ubiquitin-dependent protein breakdown, ribosome-associated ubiquitin-dependent protein catabolism, ribosome-associated ubiquitin-dependent protein degradation References: PMID:23358411 Sources: GOC:dgf Relationships: is a type of GO:0043161 Definition: The chemical reactions and pathways resulting in the breakdown of a protein or peptide encoded by an aberrant message and associated with a stalled ribosome. Degradation is initiated by the covalent attachment of a ubiquitin group, or multiple ubiquitin groups, to the ribosome-associated protein.